cyanelle envelope [GO:0033112] (CC) Relationships: is a type of plastid envelope [GO:0009526]; is part of cyanelle [GO:0009842] Definition: The double lipid bilayer enclosing the cyanelle and separating its contents from the rest of the cytoplasm; includes the intermembrane space. Sources: GOC:mah